{
  "gene_symbol": "ARL5A",
  "term_label": "vesicle-mediated transport",
  "gene": "UniProtKB:Q9Y689",
  "term_id": "GO:0016192",
  "gene_name": "ADP-ribosylation factor-like protein 5A"
}